{
  "gene_name": "Holocytochrome c-type synthase",
  "gene": "UniProtKB:P53701",
  "term_label": "Unknown biological process",
  "gene_symbol": "HCCS",
  "term_id": "UNKNOWN:0002"
}